{
  "term_id": "UNKNOWN:0002",
  "term_label": "Unknown biological process",
  "gene_name": "MYG1 exonuclease",
  "gene_symbol": "MYG1",
  "gene": "UniProtKB:Q9HB07"
}